{
  "gene_symbol": "ELF1",
  "term_label": "cell differentiation",
  "gene": "UniProtKB:P32519",
  "gene_name": "ETS-related transcription factor Elf-1",
  "term_id": "GO:0030154"
}